glomerular endothelium fenestra [GO:0036053] (cellular component) Definition: A large plasma membrane-lined circular pore that perforates the flattened glomerular endothelium and, unlike those of other fenestrated capillaries, is not spanned by diaphragms; the density and size of glomerular fenestrae account, at least in part, for the high permeability of the glomerular capillary wall to water and small solutes. References: PMID:19129259 Sources: GOC:cjm, MP:0011454 Also known as: GEnC fenestration, glomerular endothelial cell fenestration Relationships: is a type of pore complex [GO:0046930]